{
  "gene_name": "Sialidase-1",
  "gene": "UniProtKB:Q99519",
  "term_label": "exo-alpha-sialidase activity",
  "term_id": "GO:0004308",
  "gene_symbol": "NEU1"
}